{
  "gene": "UniProtKB:Q9P2J2",
  "gene_symbol": "IGSF9",
  "term_id": "GO:0007156",
  "gene_name": "Protein turtle homolog A",
  "term_label": "homophilic cell-cell adhesion"
}